cellular response to cortisone stimulus [GO:0071388] (biological process) Relationships: is a type of response to cortisone [GO:0051413]; is a type of cellular response to glucocorticoid stimulus [GO:0071385]; is a type of cellular response to alcohol [GO:0097306]; is_a GO:1901655 Sources: GOC:mah Definition: Any process that results in a change in state or activity of a cell (in terms of movement, secretion, enzyme production, gene expression, etc.) as a result of a cortisone stimulus. Cortisone is a natural glucocorticoid steroid hormone that is metabolically convertible to cortisol. Cortisone is synthesized from cholesterol in the cortex of the adrenal gland under the stimulation of adrenocorticotropin hormone (ACTH). The main physiological effect of cortisone is on carbohydrate metabolism; it can stimulate increased glucose release from the liver, increased liver glycogen synthesis, and decreased utilization of glucose by the tissues.